regulation of mitotic spindle organization [GO:0060236] (biological process) Definition: Any process that modulates the rate, frequency or extent of the assembly, arrangement of constituent parts, or disassembly of the microtubule spindle during a mitotic cell cycle. Sources: GOC:ascb_2009, GOC:dph, GOC:tb Also known as: regulation of mitotic spindle organisation, regulation of mitotic spindle organization and biogenesis Relationships: is a type of regulation of spindle organization [GO:0090224]; RO_0002211 mitotic spindle organization [GO:0007052] Subtypes: GO:0110028, regulation of mitotic spindle elongation (spindle phase three) [GO:0110162], regulation of mitotic spindle assembly [GO:1901673], GO:1904686